{
  "gene_name": "Thyroid hormone receptor alpha",
  "gene": "UniProtKB:P10827",
  "term_label": "nuclear receptor activity",
  "gene_symbol": "THRA",
  "term_id": "GO:0004879"
}